{
  "term_id": "UNKNOWN:0001",
  "gene_symbol": "ANAPC13",
  "term_label": "Unknown molecular function",
  "gene": "UniProtKB:Q9BS18",
  "gene_name": "Anaphase-promoting complex subunit 13"
}